IMP binding [GO:1902249] (molecular function) References: PMID:4314233 Sources: GOC:TermGenie, GOC:mah Definition: Binding to IMP, inosine monophosphate. Relationships: is a type of purine ribonucleotide binding [GO:0032555]; is a type of anion binding [GO:0043168]